deoxyinosine salvage [GO:0006191] (BP) Sources: GOC:jl Definition: Any process that generates deoxyinosine from derivatives of it, without de novo synthesis. Relationships: is a type of purine deoxyribonucleoside salvage [GO:0043098]; is a type of deoxyinosine biosynthetic process [GO:0046095]